{
  "term_id": "GO:0098839",
  "gene_symbol": "LRFN2",
  "term_label": "postsynaptic density membrane",
  "gene": "UniProtKB:Q9ULH4",
  "gene_name": "Leucine-rich repeat and fibronectin type-III domain-containing protein 2"
}